{
  "gene_symbol": "POLR1E",
  "gene": "UniProtKB:Q9GZS1",
  "gene_name": "DNA-directed RNA polymerase I subunit RPA49",
  "term_label": "RNA polymerase I preinitiation complex assembly",
  "term_id": "GO:0001188"
}